{
  "term_id": "UNKNOWN:0001",
  "term_label": "Unknown molecular function",
  "gene_symbol": "NPIPA2",
  "gene_name": "Nuclear pore complex-interacting protein family member A2",
  "gene": "UniProtKB:E9PIF3"
}